secretion of vasopressin involved in fast regulation of systemic arterial blood pressure [GO:0002004] (biological process) Definition: The regulated release of the hormone vasopressin into the blood stream by the hypothalamus and pituitary gland contributing to fast regulation of blood pressure. Relationships: is a type of vasopressin secretion [GO:0030103]; is part of regulation of systemic arterial blood pressure by vasopressin [GO:0001992] Sources: ISBN:0721643949 Also known as: secretion of vasopressin during fast control of blood pressure, secretion of vasopressin during fast regulation of systemic arterial blood pressure